{
  "term_label": "cellular response to lipopolysaccharide",
  "gene_name": "TNFAIP3-interacting protein 3",
  "gene": "UniProtKB:Q96KP6",
  "term_id": "GO:0071222",
  "gene_symbol": "TNIP3"
}